{
  "gene_symbol": "KAT7",
  "gene_name": "Histone acetyltransferase KAT7",
  "term_label": "nucleus",
  "gene": "UniProtKB:O95251",
  "term_id": "GO:0005634"
}